cellular response to nutrient [GO:0031670] (biological process) Definition: Any process that results in a change in state or activity of a cell (in terms of movement, secretion, enzyme production, gene expression, etc.) as a result of a nutrient stimulus. Relationships: is a type of response to nutrient [GO:0007584]; is a type of cellular response to nutrient levels [GO:0031669]; is a type of cellular response to chemical stimulus [GO:0070887] Sources: GOC:mah Subtypes: carbon catabolite regulation of transcription [GO:0045990], cellular response to methionine [GO:0061431], catabolite repression [GO:0061984], cellular response to vitamin [GO:0071295], nitrogen catabolite regulation of transcription [GO:0090293]